taurine metabolic process [GO:0019530] (BP) Also known as: taurine metabolism Subtypes: GO:0019452, taurine catabolic process [GO:0019529], GO:0042412 Relationships: is_a alkanesulfonate metabolic process [GO:0019694] Sources: GOC:jl, ISBN:0198600461 Definition: The chemical reactions and pathways involving taurine (2-aminoethanesulfonic acid), a sulphur-containing amino acid derivative important in the metabolism of fats.